pigment cell differentiation [GO:0050931] (biological process) Sources: GOC:dgh Relationships: is a type of GO:0030154; is part of developmental pigmentation [GO:0048066] Subtypes: melanocyte differentiation [GO:0030318], GO:0048772, erythrophore differentiation [GO:0048773], GO:0048774, iridophore differentiation [GO:0050935], GO:0050936, compound eye pigment cell differentiation [GO:0062056] Note: Note that the chromatophore mentioned here is distinct from the pigment bearing structure found in certain photosynthetic bacteria and cyanobacteria. It is also different from the plant chromoplast, which is also sometimes called a chromatophore. Definition: The process in which a relatively unspecialized cell acquires the specialized features of a pigmented cell, such as a melanocyte. Regulation: regulated by regulation of pigment cell differentiation [GO:0050932]; negatively regulated by negative regulation of pigment cell differentiation [GO:0050941]; positively regulated by positive regulation of pigment cell differentiation [GO:0050942] Also known as: chromatophore differentiation, pigmented cell differentiation